{
  "gene": "UniProtKB:Q7L590",
  "term_label": "DNA replication origin binding",
  "term_id": "GO:0003688",
  "gene_symbol": "MCM10",
  "gene_name": "Protein MCM10 homolog"
}